{
  "term_id": "UNKNOWN:0002",
  "gene_symbol": "RLIG1",
  "term_label": "Unknown biological process",
  "gene": "UniProtKB:Q8N999",
  "gene_name": "RNA ligase 1"
}